lanosterol synthase activity [GO:0000250] (molecular function) Also known as: 2,3-oxidosqualene sterol cyclase activity, squalene epoxidase-cyclase activity, 2,3-epoxysqualene-lanosterol cyclase activity, OSC, oxidosqualene-lanosterol cyclase activity, oxidosqualene:lanosterol cyclase activity, (S)-2,3-epoxysqualene mutase (cyclizing, lanosterol-forming), 2,3-epoxysqualene lanosterol cyclase activity, 2,3-epoxysqualene--lanosterol cyclase activity, 2,3-oxidosqualene-lanosterol cyclase activity, lanosterol 2,3-oxidosqualene cyclase activity, oxidosqualene--lanosterol cyclase activity, squalene 2,3-epoxide:lanosterol cyclase activity, squalene-2,3-oxide-lanosterol cyclase activity Definition: Catalysis of the reaction: (S)-2,3-epoxysqualene = lanosterol. This is a cyclization reaction that forms the sterol nucleus. Sources: EC:5.4.99.7, RHEA:14621 Relationships: is a type of GO:0031559